beta3-adrenergic receptor activity [GO:0015052] (MF) Definition: Combining with epinephrine or norepinephrine to initiate a change in cell activity via activation of a G protein, with pharmacological characteristics of beta3-adrenergic receptors. Also known as: beta3 adrenoceptor Relationships: is_a beta-adrenergic receptor activity [GO:0004939] Sources: GOC:mah, IUPHAR_GPCR:1274